{
  "term_label": "phospholipid translocation",
  "gene_symbol": "ANO3",
  "gene": "UniProtKB:Q9BYT9",
  "term_id": "GO:0045332",
  "gene_name": "Anoctamin-3"
}